{
  "gene_symbol": "HAUS6",
  "gene": "UniProtKB:Q7Z4H7",
  "term_id": "GO:1990498",
  "term_label": "mitotic spindle microtubule",
  "gene_name": "HAUS augmin-like complex subunit 6"
}